{
  "term_label": "L-proline biosynthetic process",
  "gene": "UniProtKB:Q96C36",
  "gene_name": "Pyrroline-5-carboxylate reductase 2",
  "term_id": "GO:0055129",
  "gene_symbol": "PYCR2"
}